{
  "gene_symbol": "KCNE1",
  "term_label": "voltage-gated potassium channel activity involved in ventricular cardiac muscle cell action potential repolarization",
  "gene": "UniProtKB:P15382",
  "gene_name": "Potassium voltage-gated channel subfamily E member 1",
  "term_id": "GO:1902282"
}